{
  "gene_name": "Putative keratin-associated protein 20-4",
  "gene": "UniProtKB:Q3LI62",
  "gene_symbol": "KRTAP20-4",
  "term_id": "UNKNOWN:0002",
  "term_label": "Unknown biological process"
}